{
  "term_id": "GO:0140861",
  "term_label": "DNA repair-dependent chromatin remodeling",
  "gene": "UniProtKB:Q9NWY4",
  "gene_symbol": "HPF1",
  "gene_name": "Histone PARylation factor 1"
}